{
  "gene_name": "Protocadherin-11 X-linked",
  "term_label": "cell adhesion molecule binding",
  "term_id": "GO:0050839",
  "gene_symbol": "PCDH11X",
  "gene": "UniProtKB:Q9BZA7"
}